{
  "gene_name": "Sorting nexin-14",
  "gene_symbol": "SNX14",
  "gene": "UniProtKB:Q9Y5W7",
  "term_label": "autophagosome maturation",
  "term_id": "GO:0097352"
}